{
  "term_label": "structural constituent of cytoskeleton",
  "gene_name": "Peripherin",
  "gene": "UniProtKB:P41219",
  "gene_symbol": "PRPH",
  "term_id": "GO:0005200"
}